{
  "term_label": "Unknown cellular component",
  "term_id": "UNKNOWN:0003",
  "gene_symbol": "BAG2",
  "gene": "UniProtKB:O95816",
  "gene_name": "BAG family molecular chaperone regulator 2"
}